{
  "gene_name": "Kinetochore-associated protein NSL1 homolog",
  "gene_symbol": "NSL1",
  "term_label": "MIS12/MIND type complex",
  "gene": "UniProtKB:Q96IY1",
  "term_id": "GO:0000444"
}